{
  "gene": "UniProtKB:Q15124",
  "term_label": "cytosol",
  "gene_symbol": "PGM5",
  "term_id": "GO:0005829",
  "gene_name": "Phosphoglucomutase-like protein 5"
}